{
  "gene_symbol": "YPEL3",
  "gene_name": "Protein yippee-like 3",
  "term_id": "UNKNOWN:0002",
  "term_label": "Unknown biological process",
  "gene": "UniProtKB:P61236"
}